{
  "term_id": "UNKNOWN:0001",
  "gene_name": "TRAF-type domain-containing protein (Fragment)",
  "gene": "UniProtKB:E9PQ42",
  "term_label": "Unknown molecular function",
  "gene_symbol": "LOC84773-CYHR1"
}